{
  "term_label": "Unknown biological process",
  "gene_name": "Serine_threonine-protein kinase SBK1",
  "gene": "UniProtKB:Q52WX2",
  "term_id": "UNKNOWN:0002",
  "gene_symbol": "SBK1"
}